{
  "term_id": "UNKNOWN:0001",
  "gene_name": "2-oxoisovalerate dehydrogenase subunit alpha, mitochondrial",
  "gene_symbol": "BCKDHA",
  "term_label": "Unknown molecular function",
  "gene": "UniProtKB:P12694"
}